{
  "gene_name": "Nociceptin receptor",
  "term_id": "GO:0019233",
  "gene": "UniProtKB:P41146",
  "term_label": "sensory perception of pain",
  "gene_symbol": "OPRL1"
}